{
  "gene": "UniProtKB:Q15031",
  "term_label": "mitochondrion",
  "gene_name": "Leucine--tRNA ligase, mitochondrial",
  "term_id": "GO:0005739",
  "gene_symbol": "LARS2"
}